{
  "term_label": "membrane raft",
  "gene_name": "Phosphoprotein associated with glycosphingolipid-enriched microdomains 1",
  "gene": "UniProtKB:Q9NWQ8",
  "term_id": "GO:0045121",
  "gene_symbol": "PAG1"
}